kidney development [GO:0001822] (biological process) Definition: The process whose specific outcome is the progression of the kidney over time, from its formation to the mature structure. The kidney is an organ that filters the blood and/or excretes the end products of body metabolism in the form of urine. Subtypes: metanephros development [GO:0001656], mesonephros development [GO:0001823], pronephros development [GO:0048793] Regulation: regulated by regulation of kidney development [GO:0090183]; positively regulated by positive regulation of kidney development [GO:0090184]; negatively regulated by negative regulation of kidney development [GO:0090185] Sources: GOC:dph, GOC:mtg_kidney_jan10, ISBN:0124020607, ISBN:0721662544 Relationships: is a type of animal organ development [GO:0048513]; is part of renal system development [GO:0072001] Also known as: nephrogenesis